{
  "gene_name": "Transcription factor E2F8",
  "term_id": "GO:0090575",
  "gene": "UniProtKB:A0AVK6",
  "gene_symbol": "E2F8",
  "term_label": "RNA polymerase II transcription regulator complex"
}